heptose 7-phosphate kinase activity [GO:0033785] (molecular function) Definition: Catalysis of the reaction: D-alpha,beta-D-heptose-7-phosphate + ATP = D-beta-D-heptose-1,7-bisphosphate + ADP. Sources: RHEA:27473 Relationships: is a type of carbohydrate kinase activity [GO:0019200] Also known as: D-alpha,beta-D-heptose 7-phosphate 1-kinase activity